{
  "gene_symbol": "SLC25A10",
  "gene_name": "Mitochondrial dicarboxylate carrier",
  "term_label": "malate transmembrane transport",
  "term_id": "GO:0071423",
  "gene": "UniProtKB:Q9UBX3"
}